{
  "gene_symbol": "WDR59",
  "term_id": "GO:0034198",
  "gene_name": "GATOR complex protein WDR59",
  "term_label": "cellular response to amino acid starvation",
  "gene": "UniProtKB:Q6PJI9"
}